{
  "gene_symbol": "ADCY8",
  "term_id": "GO:0005886",
  "gene": "UniProtKB:P40145",
  "term_label": "plasma membrane",
  "gene_name": "Adenylate cyclase type 8"
}